{
  "term_label": "Golgi apparatus",
  "gene": "UniProtKB:O60292",
  "gene_name": "Signal-induced proliferation-associated 1-like protein 3",
  "term_id": "GO:0005794",
  "gene_symbol": "SIPA1L3"
}